{
  "gene_symbol": "OR1J2",
  "gene_name": "Olfactory receptor 1J2",
  "term_label": "signal transduction",
  "term_id": "GO:0007165",
  "gene": "UniProtKB:Q8NGS2"
}